{
  "gene_name": "Polyunsaturated fatty acid lipoxygenase ALOX15B",
  "term_label": "linoleic acid metabolic process",
  "term_id": "GO:0043651",
  "gene": "UniProtKB:O15296",
  "gene_symbol": "ALOX15B"
}